{
  "gene_name": "Protein S100-A16",
  "gene_symbol": "S100A16",
  "term_id": "GO:0048306",
  "term_label": "calcium-dependent protein binding",
  "gene": "UniProtKB:Q96FQ6"
}